{
  "term_label": "alternative mRNA splicing, via spliceosome",
  "term_id": "GO:0000380",
  "gene_name": "Polyglutamine-binding protein 1",
  "gene_symbol": "PQBP1",
  "gene": "UniProtKB:O60828"
}